{
  "gene_name": "RNA-binding protein FXR2",
  "gene_symbol": "FXR2",
  "gene": "UniProtKB:P51116",
  "term_label": "translation regulator activity",
  "term_id": "GO:0045182"
}